negative regulation of keratinocyte differentiation [GO:0045617] (biological process) Sources: GOC:go_curators Also known as: down regulation of keratinocyte differentiation, down-regulation of keratinocyte differentiation, downregulation of keratinocyte differentiation, inhibition of keratinocyte differentiation Relationships: is a type of GO:0045605; is a type of regulation of keratinocyte differentiation [GO:0045616]; is a type of negative regulation of multicellular organismal process [GO:0051241]; negatively regulates keratinocyte differentiation [GO:0030216] Definition: Any process that stops, prevents, or reduces the frequency, rate or extent of keratinocyte differentiation.